{
  "term_label": "melanosome assembly",
  "gene_symbol": "HPS4",
  "term_id": "GO:1903232",
  "gene_name": "BLOC-3 complex member HPS4",
  "gene": "UniProtKB:Q9NQG7"
}